{
  "term_label": "voltage-gated potassium channel complex",
  "gene_name": "Potassium voltage-gated channel subfamily D member 2",
  "gene_symbol": "KCND2",
  "gene": "UniProtKB:Q9NZV8",
  "term_id": "GO:0008076"
}